establishment of granzyme B localization to T cell secretory granule [GO:0033381] (biological process) Definition: The directed movement of the protease granzyme B to a location within a secretory granule in a T cell. Sources: GOC:mah Also known as: establishment of granzyme B localisation in T cell secretory granule, establishment of granzyme B localization in T cell secretory granule, establishment of granzyme B localization in T lymphocyte secretory granule, establishment of granzyme B localization in T-cell secretory granule, establishment of granzyme B localization in T-lymphocyte secretory granule, T-lymphocyte secretory granule storage of granzyme B Relationships: is_a GO:0033378; is part of granzyme B localization to T cell secretory granule [GO:0033380]